positive regulation of myosin II filament assembly [GO:1905511] (biological process) Also known as: up regulation of myosin II filament assembly, up-regulation of myosin II filament assembly, upregulation of myosin II filament assembly, activation of myosin II filament assembly, activation of myosin II polymerization, positive regulation of myosin II polymerization, up regulation of myosin II polymerization, up-regulation of myosin II polymerization, upregulation of myosin II polymerization Relationships: is a type of positive regulation of protein-containing complex assembly [GO:0031334]; is a type of regulation of myosin II filament assembly [GO:0043520]; is a type of positive regulation of myosin II filament organization [GO:1904901]; positively regulates myosin II filament assembly [GO:0031036] Definition: Any process that activates or increases the frequency, rate or extent of myosin II filament assembly. References: PMID:27237792, PMID:7691416 Sources: GOC:TermGenie, GO_REF:0000058 Note: positive regulation / down regulation of the formation of a bipolar filament composed of myosin II molecules